{
  "term_label": "plasma membrane",
  "gene": "UniProtKB:O15197",
  "gene_name": "Ephrin type-B receptor 6",
  "gene_symbol": "EPHB6",
  "term_id": "GO:0005886"
}